long-term memory [GO:0007616] (biological process) Sources: ISBN:0582227089, http://hebb.mit.edu/courses/9.03/lecture4.html Definition: The memory process that deals with the storage, retrieval and modification of information a long time (typically weeks, months or years) after receiving that information. This type of memory is typically dependent on gene transcription regulated by second messenger activation. Relationships: is a type of memory [GO:0007613]